gap junction channel activity involved in cell communication by electrical coupling [GO:1903763] (molecular function) Subtypes: gap junction channel activity involved in cardiac conduction electrical coupling [GO:0086075] Also known as: innexin channel activity involved in cell communication by electrical coupling, innexin involved in cell communication by electrical coupling, connexin involved in cell communication by electrical coupling Definition: Any gap junction channel activity that is involved in cell communication by electrical coupling. References: PMID:24587307 Sources: GOC:BHF, GOC:TermGenie, GOC:mtg_cardiac_conduct_nov11, GOC:rl, GO_REF:0000061 Relationships: is a type of gap junction channel activity [GO:0005243]; BFO_0000050 GO:0010644